{
  "gene_symbol": "TRBV6-8",
  "term_id": "UNKNOWN:0001",
  "gene_name": "T cell receptor beta variable 6-8",
  "term_label": "Unknown molecular function",
  "gene": "UniProtKB:A0A0A6YYG3"
}